{
  "gene": "UniProtKB:Q9Y6E7",
  "term_label": "histone deacetylase activity",
  "gene_name": "NAD-dependent protein lipoamidase sirtuin-4, mitochondrial",
  "term_id": "GO:0004407",
  "gene_symbol": "SIRT4"
}